{
  "term_id": "UNKNOWN:0003",
  "gene_symbol": "XPNPEP2",
  "gene": "UniProtKB:O43895",
  "gene_name": "Xaa-Pro aminopeptidase 2",
  "term_label": "Unknown cellular component"
}